glucan 1,6-alpha-glucosidase activity [GO:0043896] (molecular function) Relationships: is a type of GO:0090599 Definition: Catalysis of the hydrolysis of (1->6)-alpha-D-glucosidic linkages in (1->6)-alpha-D-glucans and derived oligosaccharides. Sources: EC:3.2.1.70 Also known as: glucodextrinase, glucan-1,6-alpha-glucosidase activity, exo-1,6-alpha-glucosidase activity, exo-1,6-beta-glucosidase, glucan alpha-1,6-D-glucohydrolase activity, glucodextranase activity